{
  "gene": "UniProtKB:O43255",
  "gene_name": "E3 ubiquitin-protein ligase SIAH2",
  "term_id": "GO:0061630",
  "gene_symbol": "SIAH2",
  "term_label": "ubiquitin protein ligase activity"
}